{
  "term_id": "GO:0005737",
  "gene_symbol": "CYB5R4",
  "gene": "UniProtKB:Q7L1T6",
  "term_label": "cytoplasm",
  "gene_name": "Cytochrome b5 reductase 4"
}